negative regulation of protein localization to medial cortex [GO:0140325] (biological process) References: PMID:30853434 Definition: Any process that stops, prevents or reduces the frequency, rate or extent of protein localization to the medial cortex. Relationships: is a type of regulation of protein localization to medial cortex [GO:0106011]; is a type of negative regulation of protein localization to plasma membrane [GO:1903077]; is a type of negative regulation of protein localization to cell cortex [GO:1904777]; negatively regulates protein localization to medial cortex [GO:0071574]